positive regulation of brown fat cell differentiation [GO:0090336] (biological process) Sources: GOC:BHF Definition: Any process that increases the rate, frequency, or extent of brown fat cell differentiation. Brown fat cell differentiation is the process in which a relatively unspecialized cell acquires specialized features of a brown adipocyte, an animal connective tissue cell involved in adaptive thermogenesis. Brown adipocytes contain multiple small droplets of triglycerides and a high number of mitochondria. Relationships: is a type of positive regulation of fat cell differentiation [GO:0045600]; is a type of regulation of brown fat cell differentiation [GO:0090335]; positively regulates brown fat cell differentiation [GO:0050873]